{
  "gene": "UniProtKB:Q86XS5",
  "term_label": "extracellular matrix",
  "gene_name": "Angiopoietin-related protein 5",
  "term_id": "GO:0031012",
  "gene_symbol": "ANGPTL5"
}